{
  "gene_name": "G-protein coupled receptor 4",
  "gene": "UniProtKB:P46093",
  "term_id": "GO:0005886",
  "term_label": "plasma membrane",
  "gene_symbol": "GPR4"
}